{
  "term_label": "Unknown cellular component",
  "gene_symbol": "CCDC73",
  "gene": "UniProtKB:Q6ZRK6",
  "gene_name": "Coiled-coil domain-containing protein 73",
  "term_id": "UNKNOWN:0003"
}